{
  "term_id": "UNKNOWN:0002",
  "gene": "UniProtKB:Q96IZ2",
  "term_label": "Unknown biological process",
  "gene_name": "Androgen-dependent TFPI-regulating protein",
  "gene_symbol": "ADTRP"
}